{
  "gene_symbol": "FAM237B",
  "term_id": "UNKNOWN:0001",
  "gene_name": "Protein FAM237B",
  "term_label": "Unknown molecular function",
  "gene": "UniProtKB:A0A1B0GVD1"
}